{
  "term_id": "GO:0004016",
  "gene_name": "Adenylate cyclase type 7",
  "term_label": "adenylate cyclase activity",
  "gene_symbol": "ADCY7",
  "gene": "UniProtKB:P51828"
}